{
  "term_id": "UNKNOWN:0001",
  "gene_symbol": "KRTAP23-1",
  "gene": "UniProtKB:A1A580",
  "gene_name": "Keratin-associated protein 23-1",
  "term_label": "Unknown molecular function"
}